{
  "term_id": "UNKNOWN:0001",
  "gene_symbol": "CIAO1",
  "gene": "UniProtKB:O76071",
  "gene_name": "Probable cytosolic iron-sulfur protein assembly protein CIAO1",
  "term_label": "Unknown molecular function"
}